{
  "gene": "UniProtKB:Q96PZ2",
  "gene_name": "Serine protease FAM111A",
  "gene_symbol": "FAM111A",
  "term_id": "GO:0000785",
  "term_label": "chromatin"
}